{
  "term_id": "UNKNOWN:0003",
  "gene_name": "Bridge-like lipid transfer protein family member 3A",
  "gene_symbol": "BLTP3A",
  "gene": "UniProtKB:Q6BDS2",
  "term_label": "Unknown cellular component"
}